{
  "term_label": "DNA-binding transcription factor activity",
  "gene_name": "Zinc finger protein 282",
  "gene": "UniProtKB:Q9UDV7",
  "gene_symbol": "ZNF282",
  "term_id": "GO:0003700"
}